negative regulation of anterior/posterior axon guidance [GO:1905487] (biological process) References: PMID:16516839 Sources: GOC:TermGenie, GO_REF:0000058 Relationships: is_a negative regulation of axon guidance [GO:1902668]; is a type of regulation of anterior/posterior axon guidance [GO:1905486]; negatively regulates anterior/posterior axon guidance [GO:0033564] Also known as: down regulation of anterior-posterior axon guidance, down regulation of anterior/posterior axon guidance, down regulation of anterior/posterior axon pathfinding, down-regulation of anterior-posterior axon guidance, down-regulation of anterior/posterior axon guidance, down-regulation of anterior/posterior axon pathfinding, downregulation of anterior-posterior axon guidance, downregulation of anterior/posterior axon guidance, downregulation of anterior/posterior axon pathfinding, negative regulation of anterior-posterior axon guidance, negative regulation of anterior/posterior axon pathfinding, inhibition of anterior-posterior axon guidance, inhibition of anterior/posterior axon guidance, inhibition of anterior/posterior axon pathfinding Definition: Any process that stops, prevents or reduces the frequency, rate or extent of anterior/posterior axon guidance.